nucleosome organization [GO:0034728] (biological process) Definition: A process that is carried out at the cellular level which results in the assembly, arrangement of constituent parts, or disassembly of one or more nucleosomes. Sources: GOC:mah Also known as: nucleosome organisation Relationships: is a type of chromatin remodeling [GO:0006338]; is a type of protein-DNA complex organization [GO:0071824] Subtypes: GO:0006334, nucleosome disassembly [GO:0006337]